{
  "term_label": "DNA damage response",
  "gene": "UniProtKB:Q9BQI6",
  "term_id": "GO:0006974",
  "gene_symbol": "SLF1",
  "gene_name": "SMC5-SMC6 complex localization factor protein 1"
}